positive regulation of auxin biosynthetic process [GO:0010601] (biological process) Definition: Any process that activates or increases the frequency, rate or extent of the chemical reactions and pathways resulting in the formation of auxins, plant hormones that regulate aspects of plant growth. References: PMID:18287041 Relationships: is a type of GO:0010600; is_a GO:0046886; is a type of GO:0090355; positively regulates auxin biosynthetic process [GO:0009851]